{
  "gene_name": "Protein FAM183BP",
  "gene": "UniProtKB:Q6ZVS7",
  "term_id": "UNKNOWN:0002",
  "term_label": "Unknown biological process",
  "gene_symbol": "CFAP144P1"
}